{
  "gene": "UniProtKB:Q96K58",
  "term_id": "GO:0005634",
  "gene_name": "Zinc finger protein 668",
  "gene_symbol": "ZNF668",
  "term_label": "nucleus"
}